dimethylglycine dehydrogenase activity [GO:0047865] (molecular function) Note: Note that this was EC:1.5.99.2. Definition: Catalysis of the reaction: N,N-dimethylglycine + electron-transfer flavoprotein + H2O = sarcosine + formaldehyde + reduced electron-transfer flavoprotein. Relationships: is_a oxidoreductase activity, acting on the CH-NH group of donors, flavin as acceptor [GO:0046997] Also known as: N,N-dimethylglycine oxidase activity, N,N-dimethylglycine:(acceptor) oxidoreductase (demethylating), N,N-dimethylglycine:acceptor oxidoreductase (demethylating) Sources: EC:1.5.8.4, RHEA:52856